{
  "gene_symbol": "AJM1",
  "gene": "UniProtKB:C9J069",
  "term_id": "GO:0005886",
  "term_label": "plasma membrane",
  "gene_name": "Apical junction component 1 homolog"
}